{
  "gene_symbol": "MEF2A",
  "term_id": "GO:0042826",
  "gene_name": "Myocyte-specific enhancer factor 2A",
  "term_label": "histone deacetylase binding",
  "gene": "UniProtKB:Q02078"
}